{
  "term_id": "GO:0050890",
  "gene_name": "Tyrosine 3-monooxygenase",
  "gene": "UniProtKB:P07101",
  "term_label": "cognition",
  "gene_symbol": "TH"
}